pollen-stigma interaction [GO:0140301] (biological process) Relationships: is a type of pollen-pistil interaction [GO:0009875] Definition: The interactions (or cell to cell communication) that occur between the pollen grain (male gametophyte) and the stigmatic tissues of the female sporophyte after the pollen reaches the stigmatic papillae. References: PMID:27899537